dolichyl-phosphate-mannose-protein mannosyltransferase Pmt1p-Pmt2p dimer complex [GO:0097582] (cellular component) References: PMID:12551906 Sources: GOC:jd Relationships: is a type of dolichyl-phosphate-mannose-protein mannosyltransferase complex [GO:0031502] Also known as: Pmt1p-Pmt2p complex Definition: A protein dimer complex that possesses dolichyl-phosphate-mannose-protein mannosyltransferase activity and, in S. cerevisiae, is composed of Pmt1p-Pmt2p.